{
  "gene_symbol": "LAX1",
  "term_label": "negative regulation of T cell activation",
  "term_id": "GO:0050868",
  "gene_name": "Lymphocyte transmembrane adapter 1",
  "gene": "UniProtKB:Q8IWV1"
}